{
  "gene_name": "Zinc finger protein 37A",
  "term_id": "GO:0000981",
  "term_label": "DNA-binding transcription factor activity, RNA polymerase II-specific",
  "gene": "UniProtKB:P17032",
  "gene_symbol": "ZNF37A"
}